leg disc proximal/distal pattern formation [GO:0007479] (biological process) Relationships: is a type of proximal/distal pattern formation, imaginal disc [GO:0007449]; is a type of leg disc pattern formation [GO:0035223] Sources: GOC:bf Definition: The establishment, maintenance and elaboration of the proximal/distal axis of the leg imaginal disc, a precursor to the adult leg.